{
  "term_label": "Unknown biological process",
  "term_id": "UNKNOWN:0002",
  "gene_symbol": "CALHM1",
  "gene": "UniProtKB:Q8IU99",
  "gene_name": "Calcium homeostasis modulator protein 1"
}